{
  "gene_symbol": "FPGT",
  "term_label": "Unknown molecular function",
  "term_id": "UNKNOWN:0001",
  "gene_name": "Fucose-1-phosphate guanylyltransferase",
  "gene": "UniProtKB:O14772"
}